{
  "gene_name": "Coiled-coil domain-containing protein 184",
  "term_label": "Unknown molecular function",
  "gene": "UniProtKB:Q52MB2",
  "gene_symbol": "CCDC184",
  "term_id": "UNKNOWN:0001"
}